{
  "gene_name": "Presenilin-2",
  "gene": "UniProtKB:P49810",
  "term_label": "calcium ion homeostasis",
  "term_id": "GO:0055074",
  "gene_symbol": "PSEN2"
}